protein localization to prospore membrane [GO:1902657] (biological process) Relationships: is a type of protein localization to membrane [GO:0072657] Also known as: protein localisation in prospore membrane, protein localisation to prospore membrane, protein localization in prospore membrane, establishment of protein localisation in prospore membrane, establishment of protein localisation to prospore membrane, establishment of protein localization in prospore membrane, establishment of protein localization to prospore membrane, protein targeting to FSM, protein targeting to ascospore-type prospore membrane, protein targeting to forespore membrane, protein targeting to prospore membrane, protein-prospore membrane targeting References: PMID:24036347 Sources: GOC:TermGenie, GOC:dph, GO_REF:0000087 Regulation: regulated by regulation of protein localization to prospore membrane [GO:2001231]; positively regulated by GO:2001232 Definition: A process in which a protein is transported to, or maintained in, a location within a prospore membrane.